actomyosin, myosin complex part [GO:0042642] (cellular component) Definition: The myosin part of any complex of actin, myosin, and accessory proteins. Relationships: is a type of myosin complex [GO:0016459]; is part of actomyosin [GO:0042641] Sources: GOC:go_curators